{
  "gene_symbol": "IGKC",
  "term_label": "IgG immunoglobulin complex",
  "term_id": "GO:0071735",
  "gene": "UniProtKB:P01834",
  "gene_name": "Immunoglobulin kappa constant"
}